{
  "gene": "UniProtKB:Q9Y6P5",
  "gene_name": "Sestrin-1",
  "term_label": "cellular response to L-leucine",
  "gene_symbol": "SESN1",
  "term_id": "GO:0071233"
}